{
  "gene_name": "Peroxisomal membrane protein PMP34",
  "gene": "UniProtKB:O43808",
  "term_label": "FAD transmembrane transporter activity",
  "gene_symbol": "SLC25A17",
  "term_id": "GO:0015230"
}